{
  "term_id": "UNKNOWN:0001",
  "gene": "UniProtKB:A0A2R8YE69",
  "gene_symbol": "A0A2R8YE69",
  "gene_name": "Uncharacterized protein",
  "term_label": "Unknown molecular function"
}